{
  "gene": "UniProtKB:P56179",
  "gene_symbol": "DLX6",
  "gene_name": "Homeobox protein DLX-6",
  "term_id": "GO:0030154",
  "term_label": "cell differentiation"
}